{
  "term_label": "plasma membrane",
  "term_id": "GO:0005886",
  "gene_name": "Ras-specific guanine nucleotide-releasing factor RalGPS1",
  "gene_symbol": "RALGPS1",
  "gene": "UniProtKB:Q5JS13"
}